substrate-independent telencephalic tangential migration [GO:0021826] (BP) Subtypes: GO:0021829, substrate-independent telencephalic tangential interneuron migration [GO:0021843] References: PMID:12626695 Sources: GOC:cls, GOC:dgh, GOC:dph, GOC:jid, GO_REF:0000021 Relationships: is a type of telencephalon cell migration [GO:0022029] Definition: The process where neuronal precursors migrate tangentially in the telencephalon, primarily guided by interactions that do not require cell-cell contact.